{
  "gene": "UniProtKB:P35462",
  "gene_name": "D(3) dopamine receptor",
  "gene_symbol": "DRD3",
  "term_id": "GO:0001591",
  "term_label": "dopamine neurotransmitter receptor activity, coupled via Gi/Go"
}